{
  "gene": "UniProtKB:Q8NEN9",
  "gene_symbol": "PDZD8",
  "term_id": "GO:1990456",
  "term_label": "mitochondrion-endoplasmic reticulum membrane tethering",
  "gene_name": "PDZ domain-containing protein 8"
}